{
  "gene_name": "Transmembrane O-methyltransferase",
  "gene_symbol": "TOMT",
  "gene": "UniProtKB:Q8WZ04",
  "term_id": "GO:0016206",
  "term_label": "catechol O-methyltransferase activity"
}